{
  "term_label": "DNA-binding transcription factor activity, RNA polymerase II-specific",
  "gene_name": "Max-like protein X",
  "gene_symbol": "MLX",
  "gene": "UniProtKB:Q9UH92",
  "term_id": "GO:0000981"
}